{
  "gene_name": "Zinc finger protein 165",
  "term_label": "DNA-binding transcription factor activity, RNA polymerase II-specific",
  "gene_symbol": "ZNF165",
  "gene": "UniProtKB:P49910",
  "term_id": "GO:0000981"
}